N-acetyl-anhydromuramoyl-L-alanine amidase activity [GO:0009392] (molecular function) Sources: MetaCyc:RXN0-5225 Definition: Catalysis of the reaction: GlcNAc-1,6-anhMurNAc-L-Ala-gamma-D-Glu-DAP-D-Ala + H2O glcNAc-1,6-anhMurNAc + L-Ala-gamma-D-Glu-DAP-D-Ala. Relationships: is a type of hydrolase activity, acting on carbon-nitrogen (but not peptide) bonds [GO:0016810]